pyrimidine nucleotide import into mitochondrion [GO:1990519] (biological process) References: PMID:16194150 Definition: The process in which a pyrimidine nucleotide is transported across the mitochondrial inner membrane, into the mitochondrial matrix. Relationships: is a type of GO:0006864; is a type of pyrimidine-containing compound transmembrane transport [GO:0072531]; is a type of nucleotide transmembrane transport [GO:1901679] Also known as: mitochondrial pyrimidine nucleotide import